{
  "gene": "UniProtKB:P55001",
  "gene_name": "Microfibrillar-associated protein 2",
  "term_label": "Unknown molecular function",
  "gene_symbol": "MFAP2",
  "term_id": "UNKNOWN:0001"
}